right tetrad [GO:0097567] (CC) Definition: Set of four basal bodies found in Giardia species (trophozoite stage). It comprises the right lateral basal body pair and the right middle basal body pair (i.e. the anterior, ventral, caudal and posteriolateral basal bodies located to the left of the right nucleus of the trophozoite when viewed dorsally). References: PMID:16607022, PMID:5961344 Sources: GOC:giardia, ISBN:9780124260207 Note: Due to the asymmetric nature of the Giardia trophozoite, this term is defined spatially as the trophozoite is viewed from the dorsal side, with the two nuclei dorsal to the ventral disc, and the ventral disc toward the anterior. Relationships: is a type of GO:0110165; is part of cell projection [GO:0042995]; has part right lateral basal body pair [GO:0097564]; has part GO:0097565